{
  "gene": "UniProtKB:Q8NHV5",
  "gene_symbol": "MOSMO",
  "term_id": "GO:0005794",
  "term_label": "Golgi apparatus",
  "gene_name": "Modulator of smoothened protein"
}